{
  "gene": "UniProtKB:Q8TE54",
  "term_id": "GO:1902476",
  "gene_symbol": "SLC26A7",
  "gene_name": "Anion exchange transporter",
  "term_label": "chloride transmembrane transport"
}